{
  "gene_symbol": "UBTF",
  "gene_name": "Nucleolar transcription factor 1",
  "gene": "UniProtKB:P17480",
  "term_label": "RNA polymerase I general transcription initiation factor activity",
  "term_id": "GO:0001181"
}